negative regulation of violaceol II biosynthetic process [GO:1900717] (biological process) Definition: Any process that stops, prevents or reduces the frequency, rate or extent of violaceol II biosynthetic process. Also known as: down regulation of violaceol II anabolism, down regulation of violaceol II biosynthesis, down regulation of violaceol II biosynthetic process, down regulation of violaceol II formation, down regulation of violaceol II synthesis, down-regulation of violaceol II anabolism, down-regulation of violaceol II biosynthesis, down-regulation of violaceol II biosynthetic process, down-regulation of violaceol II formation, down-regulation of violaceol II synthesis, downregulation of violaceol II anabolism, downregulation of violaceol II biosynthesis, downregulation of violaceol II biosynthetic process, downregulation of violaceol II formation, downregulation of violaceol II synthesis, inhibition of violaceol II anabolism, inhibition of violaceol II biosynthesis, inhibition of violaceol II formation, inhibition of violaceol II synthesis, negative regulation of violaceol II anabolism, negative regulation of violaceol II biosynthesis, negative regulation of violaceol II formation, negative regulation of violaceol II synthesis, inhibition of violaceol II biosynthetic process Sources: GOC:TermGenie, GOC:di Relationships: is a type of negative regulation of secondary metabolite biosynthetic process [GO:1900377]; is a type of regulation of violaceol II biosynthetic process [GO:1900716]; negatively regulates violaceol II biosynthetic process [GO:1900593]